{
  "term_id": "GO:0004252",
  "term_label": "serine-type endopeptidase activity",
  "gene_symbol": "KLK5",
  "gene": "UniProtKB:Q9Y337",
  "gene_name": "Kallikrein-5"
}